{
  "gene_name": "Netrin-5",
  "gene": "UniProtKB:Q8WTR8",
  "gene_symbol": "NTN5",
  "term_id": "GO:0005615",
  "term_label": "extracellular space"
}